membrane reorganization involved in phagocytosis, engulfment [GO:0060098] (biological process) Relationships: is a type of plasma membrane organization [GO:0007009]; is part of phagocytosis, engulfment [GO:0006911] Sources: GOC:dph Also known as: membrane reorganisation involved in phagocytosis, engulfment Definition: The assembly and arrangement of the plasma membrane that is involved in the internalization of bacteria, immune complexes and other particulate matter or of an apoptotic cell by phagocytosis.